response to symbiotic fungus [GO:0009610] (biological process) Relationships: is a type of response to symbiont [GO:0009608]; is a type of response to fungus [GO:0009620] Also known as: response to symbiotic fungi Sources: GOC:hb, ISBN:0198506732 Definition: Any process that results in a change in state or activity of a cell or an organism (in terms of movement, secretion, enzyme production, gene expression, etc.) as a result of a stimulus from a symbiotic fungus, a fungus living in close physical association with another organism. Subtypes: detection of symbiotic fungus [GO:0009603]